{
  "gene_symbol": "SLC12A8",
  "term_label": "potassium:chloride symporter activity",
  "gene_name": "Solute carrier family 12 member 8",
  "gene": "UniProtKB:A0AV02",
  "term_id": "GO:0015379"
}